biosynthetic process [GO:0009058] (biological process) Subtypes: archaeosine-tRNA biosynthetic process [GO:0002927], GO:0006799, nitric oxide biosynthetic process [GO:0006809], GO:0008292, lipid biosynthetic process [GO:0008610], peptidyl-lysine modification to peptidyl-hypusine [GO:0008612], tRNA queuosine(34) biosynthetic process [GO:0008616], amino acid biosynthetic process [GO:0008652], macromolecule biosynthetic process [GO:0009059], amine biosynthetic process [GO:0009309], flavonoid biosynthetic process [GO:0009813], mucilage biosynthetic process [GO:0010192], carbohydrate biosynthetic process [GO:0016051], antibiotic biosynthetic process [GO:0017000], organic phosphonate biosynthetic process [GO:0032923], GO:0032964, tetrapyrrole biosynthetic process [GO:0033014], nucleobase-containing compound biosynthetic process [GO:0034654], nicotine biosynthetic process [GO:0042179], methylmercury biosynthetic process [GO:0042192], modified amino acid biosynthetic process [GO:0042398], indole-containing compound biosynthetic process [GO:0042435], hormone biosynthetic process [GO:0042446], pteridine-containing compound biosynthetic process [GO:0042559], poly(3-hydroxyalkanoate) biosynthetic process [GO:0042621], GO:0042727, peptide biosynthetic process [GO:0043043], metabolic compound salvage [GO:0043094], amide biosynthetic process [GO:0043604], sulfur compound biosynthetic process [GO:0044272], small molecule biosynthetic process [GO:0044283], GO:0044550, nucleobase biosynthetic process [GO:0046112], aldehyde biosynthetic process [GO:0046184], phenol-containing compound biosynthetic process [GO:0046189], cyanate biosynthetic process [GO:0046201], cyanide biosynthetic process [GO:0046202], Z-phenylacetaldoxime biosynthetic process [GO:0046307], phytochrome chromophore biosynthetic process [GO:0048543], GO:0051191, GO:0051559, purine-containing compound biosynthetic process [GO:0072522], pyridine-containing compound biosynthetic process [GO:0072525], pyrimidine-containing compound biosynthetic process [GO:0072528], GO:0080028, sporopollenin biosynthetic process [GO:0080110], organophosphate biosynthetic process [GO:0090407], pyocyanine biosynthetic process [GO:0106220], hydrocarbon biosynthetic process [GO:0120251], GO:0120255, GO:0140604, iron-guanylylpyridinol cofactor biosynthetic process [GO:0160300], phosphatidylinositol 4-phosphate biosynthetic process [GO:0180048], GO:1900560, GO:1900630, GO:1900999, candicidin biosynthetic process [GO:1901127], carbohydrate derivative biosynthetic process [GO:1901137], GO:1901162, tartrate biosynthetic process [GO:1901277], GO:1901288, lactone biosynthetic process [GO:1901336], poly(hydroxyalkanoate) biosynthetic process [GO:1901441], ether biosynthetic process [GO:1901503], cannabinoid biosynthetic process [GO:1901696], phosphinothricin biosynthetic process [GO:1901766], 7,8-didemethyl-8-hydroxy-5-deazariboflavin biosynthetic process [GO:1901852], tyrocidine biosynthetic process [GO:1901904], betaine aldehyde biosynthetic process [GO:1902063], GO:1902422, GO:1902756, GO:1902819, GO:1903409, methanofuran biosynthetic process [GO:2001120] Also known as: formation, anabolism, biosynthesis, synthesis, multicellular organismal biosynthetic process, single-organism biosynthetic process Relationships: is a type of metabolic process [GO:0008152] Definition: A cellular process consisting of the biochemical pathways by which a living organism synthesizes chemical substances. This typically represents the energy-requiring part of metabolism in which simpler substances are transformed into more complex ones. Regulation: regulated by GO:0009889; negatively regulated by negative regulation of biosynthetic process [GO:0009890]; RO_0002213 by positive regulation of biosynthetic process [GO:0009891] Sources: GOC:curators, ISBN:0198547684